{
  "term_label": "Unknown molecular function",
  "term_id": "UNKNOWN:0001",
  "gene_name": "T-lymphocyte activation antigen CD80",
  "gene": "UniProtKB:P33681",
  "gene_symbol": "CD80"
}